{
  "gene": "UniProtKB:P07686",
  "term_id": "GO:0016020",
  "term_label": "membrane",
  "gene_name": "Beta-hexosaminidase subunit beta",
  "gene_symbol": "HEXB"
}